{
  "gene": "UniProtKB:P46734",
  "gene_symbol": "MAP2K3",
  "gene_name": "Dual specificity mitogen-activated protein kinase kinase 3",
  "term_id": "GO:0004708",
  "term_label": "MAP kinase kinase activity"
}